regulation of viral genome replication [GO:0045069] (biological process) Relationships: is a type of regulation of viral life cycle [GO:1903900]; regulates viral genome replication [GO:0019079] Definition: Any process that modulates the frequency, rate or extent of viral genome replication. Subtypes: GO:0045070, negative regulation of viral genome replication [GO:0045071], GO:0045091 Sources: GOC:ai